{
  "gene_name": "LEM domain-containing protein 2",
  "term_label": "Unknown molecular function",
  "gene_symbol": "LEMD2",
  "gene": "UniProtKB:Q8NC56",
  "term_id": "UNKNOWN:0001"
}